mismatch repair complex binding [GO:0032404] (molecular function) Subtypes: MutLalpha complex binding [GO:0032405], GO:0032406, MutSalpha complex binding [GO:0032407], MutSbeta complex binding [GO:0032408] Sources: GOC:vk Definition: Binding to a mismatch repair complex. Relationships: is a type of GO:0044877